indoleacetylglucose-inositol O-acyltransferase activity [GO:0047194] (molecular function) Relationships: is a type of O-acyltransferase activity [GO:0008374] Also known as: 1-O-(indol-3-yl)acetyl-beta-D-glucose:myo-inositol (indol-3-yl)acetyltransferase activity, 1-O-(indol-3-ylacetyl)-beta-D-glucose:myo-inositol indole-3-ylacetyltransferase activity, indole-3-acetyl-beta-1-D-glucoside:myo-inositol indoleacetyltransferase activity Definition: Catalysis of the reaction: 1-O-(indol-3-ylacetyl)-beta-D-glucose + myo-inositol = 1L-1-O-(indol-3-yl)acetyl-myo-inositol + D-glucose. Sources: EC:2.3.1.72, RHEA:21180